N-acetyl-gamma-glutamyl-phosphate reductase activity [GO:0003942] (molecular function) Definition: Catalysis of the reaction: N-acetyl-L-glutamate 5-semialdehyde + NADP+ + phosphate = N-acetyl-5-glutamyl phosphate + NADPH + H+. Sources: RHEA:21588 Also known as: NAGSA dehydrogenase activity, N-acetyl-L-glutamate gamma-semialdehyde:NADP oxidoreductase (phosphorylating), N-acetyl-L-glutamate-5-semialdehyde:NADP+ 5-oxidoreductase (phosphorylating), N-acetyl-glutamate semialdehyde dehydrogenase activity, N-acetylglutamate 5-semialdehyde dehydrogenase activity, N-acetylglutamic gamma-semialdehyde dehydrogenase activity, reductase, acetyl-gamma-glutamyl phosphate Relationships: is a type of oxidoreductase activity, acting on the aldehyde or oxo group of donors, NAD or NADP as acceptor [GO:0016620]